{
  "gene_name": "Endothelin-converting enzyme-like 1",
  "term_id": "GO:0016485",
  "gene_symbol": "ECEL1",
  "gene": "UniProtKB:O95672",
  "term_label": "protein processing"
}